{
  "term_label": "3'-UTR-mediated mRNA stabilization",
  "term_id": "GO:0070935",
  "gene_name": "Deleted in azoospermia-like",
  "gene_symbol": "DAZL",
  "gene": "UniProtKB:Q92904"
}